{
  "gene_name": "Keratin, type I cuticular Ha1",
  "gene": "UniProtKB:Q15323",
  "gene_symbol": "KRT31",
  "term_label": "intermediate filament organization",
  "term_id": "GO:0045109"
}